{
  "gene": "UniProtKB:O15427",
  "term_label": "plasma membrane",
  "gene_symbol": "SLC16A3",
  "term_id": "GO:0005886",
  "gene_name": "Monocarboxylate transporter 4"
}